{
  "term_label": "keratin filament",
  "gene_name": "IF rod domain-containing protein",
  "term_id": "GO:0045095",
  "gene_symbol": "LOC100653049",
  "gene": "UniProtKB:A0A140TA62"
}